{
  "gene_symbol": "ABCB9",
  "gene_name": "ABC-type oligopeptide transporter ABCB9",
  "term_id": "GO:0055085",
  "gene": "UniProtKB:Q9NP78",
  "term_label": "transmembrane transport"
}